modification of postsynaptic structure [GO:0099010] (biological process) Note: This class does not cover assembly or disassembly of postsynapses, only the modification/remodelling of existing ones. Subtypes: modification of postsynaptic actin cytoskeleton [GO:0098885], modification of dendritic spine [GO:0098886] Relationships: is a type of modification of synaptic structure [GO:0099563] Definition: Any process that modifies the structure of a postsynapse. Sources: GOC:dos Also known as: synapse remodelling Regulation: regulated by GO:0099159